{
  "term_id": "GO:0007157",
  "term_label": "heterophilic cell-cell adhesion",
  "gene_symbol": "SCARF2",
  "gene_name": "Scavenger receptor class F member 2",
  "gene": "UniProtKB:Q96GP6"
}